{
  "term_label": "corticosterone 18-monooxygenase activity",
  "term_id": "GO:0047783",
  "gene": "UniProtKB:P19099",
  "gene_symbol": "CYP11B2",
  "gene_name": "Cytochrome P450 11B2, mitochondrial"
}